cardiac fibroblast cell development [GO:0060936] (BP) Subtypes: epicardium-derived cardiac fibroblast cell development [GO:0060939], neural crest-derived cardiac fibroblast cell development [GO:0060943] Relationships: is a type of cardiac cell development [GO:0055006]; is part of cardiac fibroblast cell differentiation [GO:0060935] Sources: GOC:mtg_heart Definition: The process whose specific outcome is the progression of a cardiac fibroblast over time, from its formation to the mature state. A cardiac fibroblast is a connective tissue cell of the heart which secretes an extracellular matrix rich in collagen and other macromolecules.